dedifferentiation [GO:0043696] (biological process) Relationships: is a type of developmental process [GO:0032502] Subtypes: cell dedifferentiation [GO:0043697] Definition: The process in which a specialized structure (cell, tissue or organ) loses structural or functional features that characterize it in the mature organism, or some other relatively stable phase of the organism's life history. Under certain conditions, these structures can revert back to the features of their ancestors. Sources: GOC:dph, GOC:pg